regulation of protein localization to basolateral plasma membrane [GO:1904508] (biological process) Subtypes: GO:1904509, GO:1904510 Definition: Any process that modulates the frequency, rate or extent of protein localization to basolateral plasma membrane. Relationships: is_a GO:1904375; is a type of regulation of protein localization to membrane [GO:1905475]; RO_0002211 GO:1903361 References: PMID:26115433 Sources: GOC:TermGenie, GOC:kmv, GO_REF:0000058 Also known as: regulation of protein localisation in basolateral plasma membrane, regulation of protein localisation to basolateral plasma membrane, regulation of protein localization in basolateral plasma membrane